{
  "term_label": "double-stranded DNA binding",
  "gene": "UniProtKB:Q75WM6",
  "gene_symbol": "H1-7",
  "term_id": "GO:0003690",
  "gene_name": "Testis-specific H1 histone"
}